{
  "gene": "UniProtKB:Q08170",
  "gene_symbol": "SRSF4",
  "term_id": "GO:0000381",
  "term_label": "regulation of alternative mRNA splicing, via spliceosome",
  "gene_name": "Serine_arginine-rich splicing factor 4"
}